{
  "gene_symbol": "TADA1",
  "term_id": "GO:0003713",
  "term_label": "transcription coactivator activity",
  "gene": "UniProtKB:Q96BN2",
  "gene_name": "Transcriptional adapter 1"
}